{
  "term_label": "Unknown molecular function",
  "gene": "UniProtKB:A0A0C4DH25",
  "gene_name": "Immunoglobulin kappa variable 3D-20",
  "term_id": "UNKNOWN:0001",
  "gene_symbol": "IGKV3D-20"
}